cell quiescence [GO:0044838] (biological process) Note: Note that terminally differentiated cells in higher eukaryotes are typically quiescent but metabolically active. Note that this term should not be used for direct annotation. If you are trying to make an annotation to x phase, it is likely that the correct annotation is 'regulation of x/y phase transition' or to a process which occurs during the reported phase (i.e mitotic DNA replication for mitotic S-phase). To capture the phase when a specific location or process is observed, the phase term can be used in an annotation extension (PMID:24885854) applied to a cellular component term (with the relation exists_during) or a biological process term (with the relation happens_during). Also, note that this term should not be used for direct annotation. If you are trying to make an annotation to x phase, it is likely that the correct annotation is 'regulation of x/y phase transition' or to a process which occurs during the reported phase (i.e mitotic DNA replication for mitotic S-phase). To capture the phase when a specific location or process is observed, the phase term can be used in an annotation extension (PMID:24885854) applied to a cellular component term (with the relation exists_during) or a biological process term (with the relation happens_during). Also known as: quiescence, cellular quiescence, G0 phase, cell cycle quiescence Relationships: is a type of cell cycle phase [GO:0022403] Sources: GOC:jb, GOC:mah Definition: A specialized resting state that cells enter in response to cues from the cell's environment. Quiescence is characterized by the absence of cell growth and division, by a reprogramming of global gene expression, and by changes characteristic of the organism and specific cell type. Depending on external conditions, quiescence may persist until cell death or cells may resume cell growth and division. In some cell types or under certain conditions, cellular metabolism may proceed.